{
  "term_label": "fusion of sperm to egg plasma membrane involved in single fertilization",
  "gene": "UniProtKB:W5XKT8",
  "gene_name": "Sperm acrosome membrane-associated protein 6",
  "gene_symbol": "SPACA6",
  "term_id": "GO:0007342"
}